{
  "gene": "UniProtKB:Q96M43",
  "term_label": "Unknown cellular component",
  "term_id": "UNKNOWN:0003",
  "gene_symbol": "NBPF4",
  "gene_name": "Neuroblastoma breakpoint family member 4"
}